{
  "gene_name": "Semaphorin-4F",
  "gene_symbol": "SEMA4F",
  "gene": "UniProtKB:O95754",
  "term_id": "GO:0001755",
  "term_label": "neural crest cell migration"
}